{
  "gene_symbol": "SIX3",
  "term_id": "GO:0005667",
  "gene": "UniProtKB:O95343",
  "gene_name": "Homeobox protein SIX3",
  "term_label": "transcription regulator complex"
}